flavin-containing compound metabolic process [GO:0042726] (biological process) Definition: The chemical reactions and pathways involving a flavin, any derivative of the dimethylisoalloxazine (7,8-dimethylbenzo[g]pteridine-2,4(3H,10H)-dione) skeleton, with a substituent on the 10 position. Subtypes: riboflavin metabolic process [GO:0006771], GO:0042727, flavin-containing compound catabolic process [GO:0042728], FMN metabolic process [GO:0046444], flavin adenine dinucleotide metabolic process [GO:0072387] Also known as: flavin-containing compound metabolism, riboflavin and derivative metabolic process, riboflavin and derivative metabolism, vitamin B2 and derivative metabolic process, vitamin B2 and derivative metabolism Sources: GOC:jl, GOC:mah Relationships: is a type of metabolic process [GO:0008152]